{
  "term_label": "ruffle",
  "gene_name": "Fascin-3",
  "gene_symbol": "FSCN3",
  "gene": "UniProtKB:Q9NQT6",
  "term_id": "GO:0001726"
}